lower tip-link density [GO:1990434] (cellular component) Also known as: LTLD Definition: An electron-dense plaque at the lower end of a stereocilia tip link that provides the anchor in the stereocilia membrane at the tip of the stereocilium from which the tip link rises. References: PMID:19447093 Relationships: is a type of GO:1990427